{
  "gene_name": "Unconventional myosin-Ig",
  "term_label": "endocytosis",
  "gene_symbol": "MYO1G",
  "gene": "UniProtKB:B0I1T2",
  "term_id": "GO:0006897"
}